choline:sodium symporter activity [GO:0005307] (MF) Also known as: sodium/choline symporter activity Relationships: is a type of choline transmembrane transporter activity [GO:0015220]; is a type of solute:sodium symporter activity [GO:0015370] Definition: Enables the transfer of a solute or solutes from one side of a membrane to the other according to the reaction: choline(out) + Na+(out) = choline(in) + Na+(in). Sources: TC:2.A.22.3.5